{
  "gene": "UniProtKB:Q9GZT6",
  "gene_name": "Coiled-coil domain-containing protein 90B, mitochondrial",
  "term_label": "Unknown biological process",
  "term_id": "UNKNOWN:0002",
  "gene_symbol": "CCDC90B"
}